{
  "term_id": "GO:0030154",
  "gene_symbol": "ETV2",
  "term_label": "cell differentiation",
  "gene": "UniProtKB:O00321",
  "gene_name": "ETS translocation variant 2"
}